{
  "term_id": "GO:0016020",
  "gene": "UniProtKB:P63261",
  "gene_name": "Actin, cytoplasmic 2",
  "term_label": "membrane",
  "gene_symbol": "ACTG1"
}